positive regulation of synaptic vesicle exocytosis [GO:2000302] (biological process) Subtypes: induction of synaptic vesicle exocytosis by positive regulation of presynaptic cytosolic calcium ion concentration [GO:0099703], positive regulation of calcium ion-dependent exocytosis of neurotransmitter [GO:1903235] Definition: Any process that activates or increases the frequency, rate or extent of synaptic vesicle exocytosis. Sources: GOC:obol Relationships: is a type of GO:0001956; is a type of positive regulation of regulated secretory pathway [GO:1903307]; is a type of GO:2000300; RO_0002213 synaptic vesicle exocytosis [GO:0016079]